{
  "term_id": "GO:0005615",
  "gene": "UniProtKB:P61812",
  "term_label": "extracellular space",
  "gene_name": "Transforming growth factor beta-2 proprotein",
  "gene_symbol": "TGFB2"
}